p-coumaryl alcohol transport [GO:1901140] (biological process) Definition: The directed movement of a p-coumaryl alcohol into, out of or within a cell, or between cells, by means of some agent such as a transporter or pore. Sources: GOC:TermGenie Relationships: is_a organic hydroxy compound transport [GO:0015850] Also known as: 4-hydroxycinnamyl alcohol transport